{
  "gene": "UniProtKB:O43295",
  "gene_name": "SLIT-ROBO Rho GTPase-activating protein 3",
  "gene_symbol": "SRGAP3",
  "term_label": "regulation of synapse assembly",
  "term_id": "GO:0051963"
}